isocitrate dehydrogenase (NAD+) activity [GO:0004449] (molecular function) Definition: Catalysis of the reaction: isocitrate + NAD+ = 2-oxoglutarate + CO2 + NADH. Sources: RHEA:23632 Also known as: NAD dependent isocitrate dehydrogenase activity, NAD isocitrate dehydrogenase activity, NAD isocitric dehydrogenase activity, NAD-linked isocitrate dehydrogenase activity, NAD-specific isocitrate dehydrogenase activity, isocitrate dehydrogenase (NAD) activity, isocitrate:NAD+ oxidoreductase (decarboxylating), nicotinamide adenine dinucleotide isocitrate dehydrogenase activity Relationships: is a type of GO:0004448